{
  "term_id": "UNKNOWN:0001",
  "gene": "UniProtKB:Q9Y2Y6",
  "term_label": "Unknown molecular function",
  "gene_name": "Transmembrane protein 98",
  "gene_symbol": "TMEM98"
}